{
  "gene": "UniProtKB:P81534",
  "gene_symbol": "DEFB103B",
  "term_id": "GO:0060326",
  "term_label": "cell chemotaxis",
  "gene_name": "Beta-defensin 103"
}